ends during [RO:0002093] (external)